replicative DNA transposition [GO:0098039] (biological process) Also known as: copy-and-paste transposition, replicative transposition, DNA-mediated, transpositional DNA genome replication References: PMID:10540284, PMID:1660177 Sources: GOC:bm Relationships: is a type of DNA transposition [GO:0006313]; has part GO:0006260 Definition: Process of transposition in which the existing element is replicated and one of the copies is excised and integrated at a new target site. Also referred to as copy-and-paste transposition.